{
  "term_id": "GO:0004867",
  "term_label": "serine-type endopeptidase inhibitor activity",
  "gene_name": "Serpin A11",
  "gene_symbol": "SERPINA11",
  "gene": "UniProtKB:Q86U17"
}